{
  "term_label": "termination of RNA polymerase II transcription",
  "gene_name": "RNA polymerase II subunit A C-terminal domain phosphatase SSU72 like protein 6",
  "gene": "UniProtKB:A0A1W2PR75",
  "term_id": "GO:0006369",
  "gene_symbol": "SSU72L6"
}